{
  "term_id": "GO:0006874",
  "term_label": "intracellular calcium ion homeostasis",
  "gene_symbol": "STC2",
  "gene": "UniProtKB:O76061",
  "gene_name": "Stanniocalcin-2"
}